{
  "gene_symbol": "MGAT5",
  "gene_name": "Alpha-1,6-mannosylglycoprotein 6-beta-N-acetylglucosaminyltransferase A",
  "gene": "UniProtKB:Q09328",
  "term_label": "protein N-linked glycosylation",
  "term_id": "GO:0006487"
}